{
  "term_id": "UNKNOWN:0002",
  "term_label": "Unknown biological process",
  "gene_name": "Methyltransferase N6AMT1",
  "gene_symbol": "HEMK2",
  "gene": "UniProtKB:Q9Y5N5"
}